regulation of lipid kinase activity [GO:0043550] (biological process) Sources: GOC:bf Subtypes: positive regulation of lipid kinase activity [GO:0090218] Definition: Any process that modulates the frequency, rate or extent of lipid kinase activity, the catalysis of the transfer of a phosphate group, usually from ATP, to a simple or complex lipid. Relationships: is a type of GO:0043549; regulates GO:0001727